negative regulation of interphase mitotic telomere clustering [GO:0110066] (biological process) Definition: Any process that stops, prevents, or reduces the frequency, rate or extent of mitotic telomere clustering during interphase. Relationships: is_a negative regulation of biological process [GO:0048519]; is a type of regulation of interphase mitotic telomere clustering [GO:0110065]; negatively regulates interphase mitotic telomere clustering [GO:0120110] Also known as: negative regulation of mitotic telomere clustering during interphase, telomere dispersion during interphase References: PMID:25778919 Sources: GOC:vw